{
  "gene": "UniProtKB:Q8NAP8",
  "term_id": "GO:0005634",
  "gene_name": "Zinc finger and BTB domain-containing protein 8B",
  "gene_symbol": "ZBTB8B",
  "term_label": "nucleus"
}